{
  "term_id": "UNKNOWN:0001",
  "gene_symbol": "KMT2E",
  "term_label": "Unknown molecular function",
  "gene_name": "Inactive histone-lysine N-methyltransferase 2E",
  "gene": "UniProtKB:Q8IZD2"
}